{
  "gene": "UniProtKB:Q99633",
  "term_id": "UNKNOWN:0001",
  "term_label": "Unknown molecular function",
  "gene_symbol": "PRPF18",
  "gene_name": "Pre-mRNA-splicing factor 18"
}